{
  "gene_symbol": "COL9A3",
  "term_id": "GO:0005604",
  "gene_name": "Collagen alpha-3(IX) chain",
  "term_label": "basement membrane",
  "gene": "UniProtKB:Q14050"
}